rDNA spacer replication fork barrier binding [GO:0043110] (molecular function) Definition: Binding to replication fork barriers found in rDNA spacers, sites that inhibit replication forks in the direction opposite to rDNA transcription. Also known as: RFB binding Relationships: is a type of rDNA binding [GO:0000182]; is a type of GO:0031634 Subtypes: rDNA spacer replication fork barrier binding, bending [GO:0110035] References: PMID:14645529 Sources: GOC:jl, GOC:mah